cell wall proteoglycan metabolic process [GO:0010384] (biological process) Sources: GOC:tair_curators Definition: The chemical reactions and pathways involving cell wall peptidoglycan, a group of glycoproteins that consist of a core-protein backbone O-glycosylated by one or more complex carbohydrates. Subtypes: GO:0010405 Also known as: cell wall proteoglycan metabolism Relationships: is_a GO:0006029; is a type of cell wall macromolecule metabolic process [GO:0044036]